{
  "term_id": "UNKNOWN:0002",
  "gene": "UniProtKB:Q86VE9",
  "gene_symbol": "SERINC5",
  "term_label": "Unknown biological process",
  "gene_name": "Serine incorporator 5"
}